{
  "term_id": "GO:0005789",
  "term_label": "endoplasmic reticulum membrane",
  "gene": "UniProtKB:Q9UHQ4",
  "gene_symbol": "BCAP29",
  "gene_name": "B-cell receptor-associated protein 29"
}